{
  "gene": "UniProtKB:O00116",
  "term_id": "GO:0008609",
  "gene_symbol": "AGPS",
  "term_label": "alkylglycerone-phosphate synthase activity",
  "gene_name": "Alkyldihydroxyacetonephosphate synthase, peroxisomal"
}